4-cresol dehydrogenase (hydroxylating) activity [GO:0018695] (molecular function) Relationships: is a type of GO:0016725 Also known as: 4-cresol dehydrogenase activity, 4-cresol:acceptor oxidoreductase (methyl-hydroxylating), p-cresol methylhydroxylase activity, p-cresol-(acceptor) oxidoreductase (hydroxylating) activity Sources: EC:1.17.9.1 Definition: Catalysis of the reaction: 4-cresol + acceptor + H2O = 4-hydroxybenzaldehyde + reduced acceptor.